{
  "gene": "UniProtKB:Q5TA50",
  "gene_symbol": "CPTP",
  "term_label": "ceramide 1-phosphate transfer activity",
  "gene_name": "Ceramide-1-phosphate transfer protein",
  "term_id": "GO:1902388"
}